{
  "gene_symbol": "ACTR3C",
  "gene_name": "Actin-related protein 3C",
  "term_id": "UNKNOWN:0002",
  "term_label": "Unknown biological process",
  "gene": "UniProtKB:Q9C0K3"
}